{
  "term_label": "Unknown molecular function",
  "gene_name": "Immunoglobulin kappa variable 1-9",
  "term_id": "UNKNOWN:0001",
  "gene_symbol": "IGKV1-9",
  "gene": "UniProtKB:A0A0C4DH69"
}